positive regulation of glucagon secretion [GO:0070094] (biological process) Definition: Any process that activates or increases the frequency, rate or extent of the regulated release of glucagon. Sources: GOC:BHF, GOC:mah Relationships: is a type of GO:0070092; is a type of positive regulation of peptide hormone secretion [GO:0090277]; positively regulates glucagon secretion [GO:0070091] Also known as: up regulation of glucagon secretion, up-regulation of glucagon secretion, upregulation of glucagon secretion, activation of glucagon secretion, stimulation of glucagon secretion